{
  "gene": "UniProtKB:D6RGX4",
  "term_id": "UNKNOWN:0001",
  "gene_symbol": "FAM90A26",
  "term_label": "Unknown molecular function",
  "gene_name": "Putative protein FAM90A26"
}